{
  "gene_name": "Carboxypeptidase N catalytic chain",
  "gene_symbol": "CPN1",
  "term_id": "GO:0004181",
  "gene": "UniProtKB:P15169",
  "term_label": "metallocarboxypeptidase activity"
}